{
  "gene_name": "Cyclic nucleotide-gated cation channel beta-1",
  "term_id": "GO:0005886",
  "gene_symbol": "CNGB1",
  "term_label": "plasma membrane",
  "gene": "UniProtKB:Q14028"
}